{
  "term_id": "GO:0043066",
  "term_label": "negative regulation of apoptotic process",
  "gene_name": "Alpha-crystallin A chain",
  "gene_symbol": "CRYAA",
  "gene": "UniProtKB:P02489"
}